{
  "gene_symbol": "CD44",
  "term_label": "transmembrane signaling receptor activity",
  "term_id": "GO:0004888",
  "gene_name": "CD44 antigen",
  "gene": "UniProtKB:P16070"
}